mannosylglycerate metabolic process [GO:0051478] (biological process) Subtypes: mannosylglycerate biosynthetic process [GO:0051479] Definition: The chemical reactions and pathways involving mannosylglycerate, a very common compatible solute in thermophilic and hyperthermophilic organisms. Also known as: mannosylglycerate metabolism Relationships: is a type of carbohydrate metabolic process [GO:0005975]; is a type of glycoside metabolic process [GO:0016137]; is a type of GO:0019752 References: PMID:11562374 Sources: GOC:ai